{
  "term_label": "negative regulation of G2/M transition of mitotic cell cycle",
  "gene_symbol": "PDIK1L",
  "gene_name": "Serine_threonine-protein kinase PDIK1L",
  "gene": "UniProtKB:Q8N165",
  "term_id": "GO:0010972"
}